{
  "term_label": "nucleus",
  "term_id": "GO:0005634",
  "gene_name": "Transcription factor Sp9",
  "gene": "UniProtKB:P0CG40",
  "gene_symbol": "SP9"
}